{
  "term_label": "mitochondrion",
  "term_id": "GO:0005739",
  "gene": "UniProtKB:Q9BW91",
  "gene_name": "ADP-ribose pyrophosphatase, mitochondrial",
  "gene_symbol": "NUDT9"
}